{
  "term_id": "GO:0034976",
  "gene_symbol": "P4HB",
  "term_label": "response to endoplasmic reticulum stress",
  "gene_name": "Protein disulfide-isomerase",
  "gene": "UniProtKB:P07237"
}